synaptic target recognition [GO:0008039] (biological process) Also known as: neuronal targeting Relationships: is a type of neuron recognition [GO:0008038] Sources: GOC:mah, ISBN:0878932437 Definition: The process in which a neuronal cell in a multicellular organism interprets signals produced by potential target cells, with which it may form synapses.